{
  "term_id": "GO:0005737",
  "gene": "UniProtKB:A6NGR9",
  "gene_symbol": "MROH6",
  "gene_name": "Maestro heat-like repeat-containing protein family member 6",
  "term_label": "cytoplasm"
}